regulation of meiotic chromosome separation [GO:1905132] (biological process) Relationships: is a type of regulation of chromosome separation [GO:1905818]; is a type of GO:2000241; RO_0002211 meiotic chromosome separation [GO:0051307] References: PMID:15620645 Sources: GOC:TermGenie, GOC:vw, GO_REF:0000058 Also known as: regulation of chromosome separation during meiosis, regulation of meiotic chromosome resolution Definition: Any process that modulates the frequency, rate or extent of meiotic chromosome separation. Subtypes: regulation of metaphase/anaphase transition of meiotic cell cycle [GO:1902102], negative regulation of meiotic chromosome separation [GO:1905133], GO:1905134